{
  "term_id": "GO:0035005",
  "gene_symbol": "PIK3C2G",
  "gene_name": "Phosphatidylinositol 3-kinase C2 domain-containing subunit gamma",
  "term_label": "1-phosphatidylinositol-4-phosphate 3-kinase activity",
  "gene": "UniProtKB:O75747"
}